{
  "gene": "UniProtKB:Q6Q788",
  "gene_name": "Apolipoprotein A-V",
  "term_label": "phosphatidylcholine-sterol O-acyltransferase activator activity",
  "term_id": "GO:0060228",
  "gene_symbol": "APOA5"
}